{
  "gene": "UniProtKB:Q8IVF5",
  "term_id": "GO:0050772",
  "gene_name": "Rho guanine nucleotide exchange factor TIAM2",
  "gene_symbol": "TIAM2",
  "term_label": "positive regulation of axonogenesis"
}